{
  "term_id": "GO:0000981",
  "gene_symbol": "ANHX",
  "gene_name": "Anomalous homeobox protein",
  "gene": "UniProtKB:E9PGG2",
  "term_label": "DNA-binding transcription factor activity, RNA polymerase II-specific"
}